{
  "gene_name": "Sialidase-3",
  "gene": "UniProtKB:Q9UQ49",
  "gene_symbol": "NEU3",
  "term_label": "lysosome",
  "term_id": "GO:0005764"
}